{
  "gene": "UniProtKB:Q8IYT8",
  "term_id": "GO:0005829",
  "term_label": "cytosol",
  "gene_symbol": "ULK2",
  "gene_name": "Serine_threonine-protein kinase ULK2"
}